{
  "term_label": "Unknown biological process",
  "gene": "UniProtKB:Q9UPU7",
  "term_id": "UNKNOWN:0002",
  "gene_name": "TBC1 domain family member 2B",
  "gene_symbol": "TBC1D2B"
}